vernalization response [GO:0010048] (biological process) Regulation: RO_0002211 by regulation of vernalization response [GO:0010219]; positively regulated by positive regulation of vernalization response [GO:0010220]; negatively regulated by negative regulation of vernalization response [GO:0010221] Relationships: is a type of response to cold [GO:0009409] Sources: GOC:tair_curators, ISBN:0521591392 Definition: The process of thermal induction in plants in which flowering is promoted by exposure to low temperatures.